{
  "gene_name": "Putative uncharacterized protein PRO2289",
  "gene_symbol": "PRO2289",
  "gene": "UniProtKB:Q9P1D8",
  "term_label": "Unknown molecular function",
  "term_id": "UNKNOWN:0001"
}